{
  "term_label": "Unknown molecular function",
  "gene_name": "Kinetochore protein NDC80 homolog",
  "gene_symbol": "NDC80",
  "gene": "UniProtKB:O14777",
  "term_id": "UNKNOWN:0001"
}